{
  "term_id": "GO:0030111",
  "gene_name": "Serine_threonine-protein kinase STK11",
  "gene": "UniProtKB:Q15831",
  "gene_symbol": "STK11",
  "term_label": "regulation of Wnt signaling pathway"
}